{
  "gene_name": "Receptor activity-modifying protein 1",
  "gene": "UniProtKB:O60894",
  "gene_symbol": "RAMP1",
  "term_id": "GO:0007186",
  "term_label": "G protein-coupled receptor signaling pathway"
}